regulation of thermomorphogenesis [GO:0140920] (biological process) References: PMID:27250752 Subtypes: negative regulation of thermomorphogenesis [GO:0140921], GO:0140922 Relationships: is a type of regulation of post-embryonic development [GO:0048580]; is a type of GO:0048583; regulates thermomorphogenesis [GO:0140919] Definition: Any process that modulates the frequency, rate or extent of thermomorphogenesis.